{
  "term_label": "glycine transport",
  "gene": "UniProtKB:Q495M3",
  "term_id": "GO:0015816",
  "gene_name": "Proton-coupled amino acid transporter 2",
  "gene_symbol": "SLC36A2"
}